{
  "gene": "UniProtKB:Q8TDM6",
  "term_label": "Unknown molecular function",
  "term_id": "UNKNOWN:0001",
  "gene_name": "Disks large homolog 5",
  "gene_symbol": "DLG5"
}